regulation of t-SNARE clustering [GO:1904032] (biological process) Subtypes: GO:1904033, positive regulation of t-SNARE clustering [GO:1904034] Relationships: is a type of GO:1905475; regulates t-SNARE clustering [GO:1990656] References: PMID:22528485 Sources: GOC:TermGenie, GO_REF:0000058 Definition: Any process that modulates the frequency, rate or extent of t-SNARE clustering.